{
  "term_label": "phosphatidylinositol-mediated signaling",
  "term_id": "GO:0048015",
  "gene_symbol": "PI4KA",
  "gene": "UniProtKB:P42356",
  "gene_name": "Phosphatidylinositol 4-kinase alpha"
}